trihydroxyferuloyl spermidine O-methyltransferase activity [GO:0080012] (molecular function) References: PMID:18557837 Relationships: is a type of O-methyltransferase activity [GO:0008171] Also known as: N1,N5,N10-tris-(5-hydroxyferuloyl)spermidine O-methyltransferase activity Definition: Catalysis of the reaction: trihydroxyferuloyl spermidine + S-adenosyl-L-methionine = dihydroxyferuloyl-sinapoyl spermidine + S-adenosyl-L-homocysteine + H+.